{
  "gene": "UniProtKB:Q14003",
  "gene_symbol": "KCNC3",
  "gene_name": "Potassium voltage-gated channel subfamily C member 3",
  "term_id": "GO:0042734",
  "term_label": "presynaptic membrane"
}